{
  "gene_symbol": "PCSK5",
  "term_label": "Golgi membrane",
  "gene": "UniProtKB:Q92824",
  "gene_name": "Proprotein convertase subtilisin_kexin type 5",
  "term_id": "GO:0000139"
}